{
  "gene_name": "Phosphate-regulating neutral endopeptidase PHEX",
  "gene": "UniProtKB:P78562",
  "term_id": "GO:0004222",
  "term_label": "metalloendopeptidase activity",
  "gene_symbol": "PHEX"
}